{
  "term_id": "GO:0005634",
  "gene_name": "Estrogen receptor",
  "term_label": "nucleus",
  "gene": "UniProtKB:P03372",
  "gene_symbol": "ESR1"
}